{
  "gene_symbol": "POLA1",
  "gene_name": "DNA polymerase alpha catalytic subunit",
  "term_id": "GO:0003688",
  "gene": "UniProtKB:P09884",
  "term_label": "DNA replication origin binding"
}